{
  "term_label": "piecemeal microautophagy of the nucleus",
  "gene_name": "Serine_threonine-protein kinase ULK3",
  "gene": "UniProtKB:Q6PHR2",
  "gene_symbol": "ULK3",
  "term_id": "GO:0034727"
}